{
  "term_label": "nuclear speck",
  "gene": "UniProtKB:Q9BY77",
  "gene_name": "Polymerase delta-interacting protein 3",
  "gene_symbol": "POLDIP3",
  "term_id": "GO:0016607"
}